{
  "term_id": "GO:0030593",
  "gene_name": "C-X-C chemokine receptor type 1",
  "term_label": "neutrophil chemotaxis",
  "gene_symbol": "CXCR1",
  "gene": "UniProtKB:P25024"
}